GDP-glucosidase activity [GO:0047917] (molecular function) Definition: Catalysis of the reaction: GDP-D-glucose + H2O = D-glucose + GDP + H+. Sources: EC:3.2.1.42, RHEA:15049 Also known as: GDP-glucose glucohydrolase activity, GDPglucose glucohydrolase activity, GDPglucosidase activity, guanosine diphosphate D-glucose glucohydrolase activity, guanosine diphosphoglucosidase activity Relationships: is a type of glucosidase activity [GO:0015926]